{
  "term_id": "GO:0019731",
  "gene_name": "Angiogenin",
  "gene_symbol": "ANG",
  "gene": "UniProtKB:P03950",
  "term_label": "antibacterial humoral response"
}